UTP:arabinose-1-phosphate uridylyltransferase activity [GO:0010491] (molecular function) References: PMID:17341835 Relationships: is a type of GO:0051748 Definition: Catalysis of the reaction: alpha-L-arabinose 1-phosphate + UTP = UDP-L-arabinose + diphosphate.